soyasapogenol B glucuronosyltransferase activity [GO:0102793] (molecular function) Sources: EC:2.4.1.262, GOC:pz Relationships: is a type of hexosyltransferase activity [GO:0016758] Definition: Catalysis of the reaction: UDP-alpha-D-glucuronate + soyasapogenol B = H+ + UDP + soyasapogenol B 3-O-beta-glucuronate.